{
  "gene_name": "D-ribitol-5-phosphate cytidylyltransferase",
  "term_id": "GO:0047349",
  "gene_symbol": "CRPPA",
  "gene": "UniProtKB:A4D126",
  "term_label": "D-ribitol-5-phosphate cytidylyltransferase activity"
}